{
  "gene_symbol": "PNLDC1",
  "gene_name": "Poly(A)-specific ribonuclease PNLDC1",
  "gene": "UniProtKB:Q8NA58",
  "term_label": "priRNA 3'-end processing",
  "term_id": "GO:1990431"
}